{
  "gene_name": "SPARC-like protein 1",
  "term_label": "calcium ion binding",
  "term_id": "GO:0005509",
  "gene_symbol": "SPARCL1",
  "gene": "UniProtKB:Q14515"
}